{
  "gene_name": "CUGBP Elav-like family member 5",
  "term_label": "mRNA splice site recognition",
  "term_id": "GO:0006376",
  "gene": "UniProtKB:Q8N6W0",
  "gene_symbol": "CELF5"
}